{
  "term_label": "nucleic acid binding",
  "term_id": "GO:0003676",
  "gene_symbol": "YBX3",
  "gene_name": "Y-box-binding protein 3",
  "gene": "UniProtKB:P16989"
}